{
  "gene_symbol": "TAP1",
  "gene_name": "Antigen peptide transporter 1",
  "gene": "UniProtKB:Q03518",
  "term_label": "membrane",
  "term_id": "GO:0016020"
}